{
  "term_id": "GO:0030992",
  "gene_symbol": "IFT81",
  "gene": "UniProtKB:Q8WYA0",
  "term_label": "intraciliary transport particle B",
  "gene_name": "Intraflagellar transport protein 81 homolog"
}